{
  "term_label": "positive regulation of T cell mediated immune response to tumor cell",
  "term_id": "GO:0002842",
  "gene_symbol": "FBXO38",
  "gene_name": "F-box only protein 38",
  "gene": "UniProtKB:Q6PIJ6"
}